positive regulation of intralumenal vesicle formation [GO:1905367] (biological process) References: PMID:26911690 Sources: GOC:PARL, GOC:TermGenie, GOC:bc, GO_REF:0000058 Definition: Any process that activates or increases the frequency, rate or extent of intralumenal vesicle formation. Relationships: is a type of positive regulation of transport [GO:0051050]; is a type of positive regulation of endosome organization [GO:1904980]; is a type of GO:1905365; positively regulates intralumenal vesicle formation [GO:0070676] Also known as: positive regulation of endosome membrane budding, up regulation of endosome membrane budding, up regulation of intralumenal vesicle formation, up-regulation of endosome membrane budding, up-regulation of intralumenal vesicle formation, upregulation of endosome membrane budding, upregulation of intralumenal vesicle formation, activation of endosome membrane budding, activation of intralumenal vesicle formation